{
  "gene_name": "Low affinity immunoglobulin gamma Fc region receptor II-a",
  "term_id": "GO:0050766",
  "gene": "UniProtKB:P12318",
  "term_label": "positive regulation of phagocytosis",
  "gene_symbol": "FCGR2A"
}